{
  "term_id": "GO:0030154",
  "gene_symbol": "NR2C2",
  "gene_name": "Nuclear receptor subfamily 2 group C member 2",
  "gene": "UniProtKB:P49116",
  "term_label": "cell differentiation"
}